negative regulation of nuclear-transcribed mRNA catabolic process, deadenylation-dependent decay [GO:1900152] (biological process) Also known as: down regulation of deadenylation-dependent mRNA decay, down regulation of mRNA breakdown, deadenylation-dependent decay, down regulation of mRNA catabolic process, deadenylation-dependent, down regulation of mRNA catabolic process, deadenylylation-dependent, down regulation of mRNA catabolism, deadenylation-dependent, down regulation of mRNA catabolism, deadenylylation-dependent, down regulation of mRNA degradation, deadenylation-dependent decay, down regulation of nuclear mRNA catabolic process, deadenylation-dependent decay, down regulation of nuclear-transcribed mRNA catabolic process, deadenylation-dependent decay, down-regulation of deadenylation-dependent mRNA decay, down-regulation of mRNA breakdown, deadenylation-dependent decay, down-regulation of mRNA catabolic process, deadenylation-dependent, down-regulation of mRNA catabolic process, deadenylylation-dependent, down-regulation of mRNA catabolism, deadenylation-dependent, down-regulation of mRNA catabolism, deadenylylation-dependent, down-regulation of mRNA degradation, deadenylation-dependent decay, down-regulation of nuclear mRNA catabolic process, deadenylation-dependent decay, down-regulation of nuclear-transcribed mRNA catabolic process, deadenylation-dependent decay, downregulation of deadenylation-dependent mRNA decay, downregulation of mRNA breakdown, deadenylation-dependent decay, downregulation of mRNA catabolic process, deadenylation-dependent, downregulation of mRNA catabolic process, deadenylylation-dependent, downregulation of mRNA catabolism, deadenylation-dependent, downregulation of mRNA catabolism, deadenylylation-dependent, downregulation of mRNA degradation, deadenylation-dependent decay, downregulation of nuclear mRNA catabolic process, deadenylation-dependent decay, downregulation of nuclear-transcribed mRNA catabolic process, deadenylation-dependent decay, negative regulation of deadenylation-dependent mRNA decay, negative regulation of mRNA breakdown, deadenylation-dependent decay, negative regulation of mRNA catabolic process, deadenylation-dependent, negative regulation of mRNA catabolic process, deadenylylation-dependent, negative regulation of mRNA catabolism, deadenylation-dependent, negative regulation of mRNA catabolism, deadenylylation-dependent, negative regulation of mRNA degradation, deadenylation-dependent decay, negative regulation of nuclear mRNA catabolic process, deadenylation-dependent decay, inhibition of deadenylation-dependent mRNA decay, inhibition of mRNA breakdown, deadenylation-dependent decay, inhibition of mRNA catabolic process, deadenylation-dependent, inhibition of mRNA catabolic process, deadenylylation-dependent, inhibition of mRNA catabolism, deadenylation-dependent, inhibition of mRNA catabolism, deadenylylation-dependent, inhibition of mRNA degradation, deadenylation-dependent decay, inhibition of nuclear mRNA catabolic process, deadenylation-dependent decay, inhibition of nuclear-transcribed mRNA catabolic process, deadenylation-dependent decay Relationships: is a type of regulation of nuclear-transcribed mRNA catabolic process, deadenylation-dependent decay [GO:1900151]; is a type of negative regulation of mRNA catabolic process [GO:1902373]; RO_0002212 nuclear-transcribed mRNA catabolic process, deadenylation-dependent decay [GO:0000288] Subtypes: negative regulation of nuclear-transcribed mRNA poly(A) tail shortening [GO:0060212] Sources: GOC:TermGenie, GOC:mcc Definition: Any process that stops, prevents or reduces the frequency, rate or extent of nuclear-transcribed mRNA catabolic process, deadenylation-dependent decay.